establishment of mitotic spindle orientation [GO:0000132] (biological process) Subtypes: establishment of mitotic spindle orientation involved in growth plate cartilage chondrocyte division [GO:0003425] Relationships: is a type of establishment of mitotic spindle localization [GO:0040001]; is a type of establishment of spindle orientation [GO:0051294] Also known as: establishment of spindle orientation involved in mitotic cell cycle, mitotic spindle orientation, orienting of mitotic spindle, establishment of spindle orientation during mitosis Definition: A cell cycle process that sets the alignment of mitotic spindle relative to other cellular structures. Sources: GOC:ems